{
  "gene_symbol": "KIFAP3",
  "term_label": "cilium organization",
  "gene_name": "Kinesin-associated protein 3",
  "gene": "UniProtKB:Q92845",
  "term_id": "GO:0044782"
}